{
  "gene_symbol": "MTMR8",
  "gene_name": "Myotubularin-related protein 8",
  "gene": "UniProtKB:Q96EF0",
  "term_label": "phosphatidylinositol dephosphorylation",
  "term_id": "GO:0046856"
}